regulation of L-proline import across plasma membrane [GO:1905735] (biological process) Definition: Any process that modulates the frequency, rate or extent of L-proline import across plasma membrane. Subtypes: GO:1905736, GO:1905737 References: PMID:24344203 Sources: GOC:TermGenie, GO_REF:0000058 Relationships: is a type of regulation of proline transport [GO:0070881]; is a type of GO:1902834; regulates L-proline import across plasma membrane [GO:1904271]